{
  "gene_symbol": "KCNH6",
  "term_label": "regulation of heart rate by cardiac conduction",
  "gene": "UniProtKB:Q9H252",
  "term_id": "GO:0086091",
  "gene_name": "Potassium voltage-gated channel subfamily H member 6"
}